{
  "gene_name": "Potassium voltage-gated channel subfamily C member 2",
  "gene_symbol": "KCNC2",
  "gene": "UniProtKB:Q96PR1",
  "term_label": "voltage-gated potassium channel complex",
  "term_id": "GO:0008076"
}